{
  "gene_symbol": "MEOX2",
  "term_label": "regulation of transcription by RNA polymerase II",
  "gene_name": "Homeobox protein MOX-2",
  "gene": "UniProtKB:P50222",
  "term_id": "GO:0006357"
}